organic hydroxy compound transport [GO:0015850] (biological process) Subtypes: serotonin transport [GO:0006837], bile acid and bile salt transport [GO:0015721], lactate transport [GO:0015727], GO:0015731, shikimate transmembrane transport [GO:0015733], polyol transmembrane transport [GO:0015791], myo-inositol transport [GO:0015798], propane 1,3-diol transport [GO:0015799], cycloheximide transport [GO:0015901], GO:0015903, GO:0015904, sterol transport [GO:0015918], pyridoxal transport [GO:0031920], pyridoxal phosphate transport [GO:0031921], pyridoxamine transport [GO:0031922], pyridoxine transport [GO:0031923], myo-inositol phosphate transport [GO:0033271], hydroxyectoine transmembrane transport [GO:0033308], ethanolamine transport [GO:0034229], GO:0034633, isopropylmalate transport [GO:0034659], aldosterone secretion [GO:0035932], corticosterone secretion [GO:0035934], GO:0035936, estradiol secretion [GO:0035938], GO:0035942, GO:0035943, 3-hydroxyphenylpropionic acid transmembrane transport [GO:0042920], enterobactin transport [GO:0042930], chrysobactin transport [GO:0042932], GO:0042935, GO:0042948, cortisol secretion [GO:0043400], catecholamine transport [GO:0051937], octopamine secretion [GO:0061539], tyramine secretion [GO:0061545], abscisic acid transport [GO:0080168], doxorubicin transport [GO:1900753], 4-hydroxyphenylacetate transport [GO:1900754], GO:1900866, p-coumaryl alcohol transport [GO:1901140] Definition: The directed movement of an organic hydroxy compound (organic alcohol) into, out of or within a cell, or between cells, by means of some agent such as a transporter or pore. An organic hydroxy compound is an organic compound having at least one hydroxy group attached to a carbon atom. Relationships: is a type of GO:0006810 Also known as: organic alcohol transport Sources: GOC:ai